siRNA binding [GO:0035197] (molecular function) Also known as: small interfering RNA binding References: PMID:15066275, PMID:15066283 Definition: Binding to a small interfering RNA, a 21-23 nucleotide RNA that is processed from double stranded RNA (dsRNA) by an RNAse enzyme. Relationships: is a type of regulatory RNA binding [GO:0061980]